{
  "term_label": "plasma membrane",
  "gene_name": "Ephrin-A3",
  "gene": "UniProtKB:P52797",
  "gene_symbol": "EFNA3",
  "term_id": "GO:0005886"
}